{
  "gene": "UniProtKB:Q8TCT9",
  "term_label": "signal peptide processing",
  "gene_name": "Minor histocompatibility antigen H13",
  "gene_symbol": "HM13",
  "term_id": "GO:0006465"
}